{
  "term_label": "ubiquitin protein ligase binding",
  "term_id": "GO:0031625",
  "gene": "UniProtKB:Q13619",
  "gene_symbol": "CUL4A",
  "gene_name": "Cullin-4A"
}